positive regulation of syncytial blastoderm mitotic cell cycle [GO:0046004] (biological process) Also known as: positive regulation of progression through syncytial blastoderm mitotic cell cycle, positive regulation of syncytial blastoderm cell cycle progression, up regulation of progression through syncytial blastoderm mitotic cell cycle, up-regulation of progression through syncytial blastoderm mitotic cell cycle, upregulation of progression through syncytial blastoderm mitotic cell cycle, activation of progression through syncytial blastoderm mitotic cell cycle, stimulation of progression through syncytial blastoderm mitotic cell cycle Sources: GOC:dph, GOC:go_curators, GOC:tb Relationships: is a type of regulation of syncytial blastoderm mitotic cell cycle [GO:0007348]; is a type of positive regulation of mitotic cell cycle, embryonic [GO:0045977]; RO_0002213 syncytial blastoderm mitotic cell cycle [GO:0035186] Definition: Any process that activates or increases the rate or extent of progression through the syncytial blastoderm mitotic cell cycle.